corticosterone 18-monooxygenase activity [GO:0047783] (molecular function) Sources: EC:1.14.15.5 Definition: Catalysis of the reaction: corticosterone + reduced adrenal ferredoxin + O2 = 18-hydroxycorticosterone + oxidized adrenal ferredoxin + H2O. Also known as: corticosterone 18-hydroxylase activity, corticosterone methyl oxidase activity, corticosterone,reduced-adrenal-ferredoxin:oxygen oxidoreductase (18-hydroxylating) Relationships: is a type of oxidoreductase activity, acting on paired donors, with incorporation or reduction of molecular oxygen, reduced iron-sulfur protein as one donor, and incorporation of one atom of oxygen [GO:0016713]